regulation of sterol biosynthetic process [GO:0106118] (biological process) Relationships: is a type of GO:0050810; regulates sterol biosynthetic process [GO:0016126] References: PMID:16459310 Sources: GOC:BHF, GOC:BHF_miRNA, GOC:rph Subtypes: regulation of ergosterol biosynthetic process [GO:0032443], regulation of cholesterol biosynthetic process [GO:0045540], negative regulation of sterol biosynthetic process [GO:0106119], positive regulation of sterol biosynthetic process [GO:0106120] Definition: Any process that modulates the frequency, rate or extent of a sterol biosynthetic process.